{
  "gene": "UniProtKB:Q9GZS0",
  "term_label": "dynein heavy chain binding",
  "gene_symbol": "DNAI2",
  "gene_name": "Dynein axonemal intermediate chain 2",
  "term_id": "GO:0045504"
}